{
  "term_label": "apical plasma membrane",
  "gene_symbol": "RAPGEF6",
  "gene_name": "Rap guanine nucleotide exchange factor 6",
  "gene": "UniProtKB:Q8TEU7",
  "term_id": "GO:0016324"
}